{
  "gene": "UniProtKB:Q86X02",
  "term_id": "UNKNOWN:0001",
  "gene_symbol": "CDR2L",
  "gene_name": "Cerebellar degeneration-related protein 2-like",
  "term_label": "Unknown molecular function"
}